appendage segmentation [GO:0035285] (BP) Relationships: is_a segmentation [GO:0035282]; is part of appendage morphogenesis [GO:0035107] References: PMID:10357895 Definition: Division of an appendage, an organ or part that is attached to the main body of an organism, into a series of semi-repetitive parts or segments. Most arthropod appendages, such as the legs and antennae, are visibly segmented. Subtypes: imaginal disc-derived leg segmentation [GO:0036011]